{
  "term_id": "UNKNOWN:0001",
  "gene_name": "Circadian clock protein PASD1",
  "term_label": "Unknown molecular function",
  "gene": "UniProtKB:Q8IV76",
  "gene_symbol": "PASD1"
}